{
  "term_id": "GO:0072686",
  "gene": "UniProtKB:Q96BD8",
  "term_label": "mitotic spindle",
  "gene_symbol": "SKA1",
  "gene_name": "Spindle and kinetochore-associated protein 1"
}